{
  "term_id": "GO:0008360",
  "term_label": "regulation of cell shape",
  "gene": "UniProtKB:Q6NZY7",
  "gene_symbol": "CDC42EP5",
  "gene_name": "Cdc42 effector protein 5"
}